{
  "gene_symbol": "C3P1",
  "gene_name": "Putative protein C3P1",
  "term_label": "Unknown cellular component",
  "gene": "UniProtKB:Q6ZMU1",
  "term_id": "UNKNOWN:0003"
}